viral life cycle [GO:0019058] (biological process) Definition: A set of processes which all viruses follow to ensure survival; includes attachment and entry of the virus particle, decoding of genome information, translation of viral mRNA by host ribosomes, genome replication, and assembly and release of viral particles containing the genome. Also known as: viral assembly, maturation, egress, and release, lytic viral life cycle, viral infectious cycle, viral replication Relationships: is a type of viral process [GO:0016032] Sources: ISBN:1555811272 Regulation: regulated by GO:1903900; RO_0002212 by negative regulation of viral life cycle [GO:1903901]; RO_0002213 by positive regulation of viral life cycle [GO:1903902]